{
  "term_label": "regulation of transcription by RNA polymerase II",
  "gene_symbol": "ZNF556",
  "gene_name": "Zinc finger protein 556",
  "gene": "UniProtKB:Q9HAH1",
  "term_id": "GO:0006357"
}